{
  "term_id": "GO:0034551",
  "gene_symbol": "UQCC4",
  "gene": "UniProtKB:Q4G0I0",
  "gene_name": "Ubiquinol-cytochrome-c reductase complex assembly factor 4",
  "term_label": "mitochondrial respiratory chain complex III assembly"
}